{
  "term_id": "GO:0048205",
  "gene_symbol": "TMED9",
  "term_label": "COPI coating of Golgi vesicle",
  "gene_name": "Transmembrane emp24 domain-containing protein 9",
  "gene": "UniProtKB:Q9BVK6"
}